{
  "term_label": "Unknown molecular function",
  "gene_symbol": "TMEM267",
  "gene": "UniProtKB:Q0VDI3",
  "term_id": "UNKNOWN:0001",
  "gene_name": "Transmembrane protein 267"
}